positive regulation of GTP binding [GO:1904426] (biological process) Also known as: up regulation of GTP binding, up-regulation of GTP binding, upregulation of GTP binding, activation of GTP binding Definition: Any process that activates or increases the frequency, rate or extent of GTP binding. Relationships: is_a GO:0051099; RO_0002213 GO:0005525 References: PMID:19066305, PMID:21454546 Sources: GOC:TermGenie, GO_REF:0000059